flavin-dependent sulfhydryl oxidase activity [GO:0016971] (molecular function) Also known as: flavin-linked sulfhydryl oxidase activity References: PMID:10899311, PMID:19679655, PMID:35495482 Relationships: is a type of protein-disulfide reductase activity [GO:0015035]; is a type of thiol oxidase activity [GO:0016972] Definition: Catalysis of the reaction: [protein]-dithiol + O2 = [protein]-disulfide + H2O2 using FAD as a cofactor, leading to formation of disulfide bridges in proteins.